{
  "term_id": "GO:0008093",
  "gene_symbol": "ANK2",
  "gene": "UniProtKB:Q01484",
  "gene_name": "Ankyrin-2",
  "term_label": "cytoskeletal anchor activity"
}